{
  "term_label": "nucleus",
  "term_id": "GO:0005634",
  "gene_name": "Neurite extension and migration factor",
  "gene_symbol": "NEXMIF",
  "gene": "UniProtKB:Q5QGS0"
}